{
  "gene_symbol": "REV1",
  "term_label": "DNA-directed DNA polymerase activity",
  "gene_name": "DNA repair protein REV1",
  "term_id": "GO:0003887",
  "gene": "UniProtKB:Q9UBZ9"
}